bulbus arteriosus development [GO:0003232] (BP) Relationships: is a type of cardiac chamber development [GO:0003205] Sources: GOC:mtg_heart Definition: The process whose specific outcome is the progression of the bulbus arteriosus over time, from its formation to the mature structure. The bulbus arteriosus is an elastic heart chamber.